{
  "term_label": "3'-phosphoadenosine 5'-phosphosulfate transport",
  "term_id": "GO:0046963",
  "gene": "UniProtKB:Q9H1N7",
  "gene_symbol": "SLC35B3",
  "gene_name": "Adenosine 3'-phospho 5'-phosphosulfate transporter 2"
}